{
  "gene_symbol": "LHFPL6",
  "term_id": "UNKNOWN:0001",
  "gene": "UniProtKB:Q9Y693",
  "gene_name": "LHFPL tetraspan subfamily member 6 protein",
  "term_label": "Unknown molecular function"
}